DNA strand exchange inhibitor activity [GO:0140620] (molecular function) References: PMID:33493431 Definition: Binds to and stops, prevents or reduces a DNA strand exchange activity. Relationships: is a type of enzyme inhibitor activity [GO:0004857]; negatively regulates GO:0000150